spongiotrophoblast layer developmental growth [GO:0090214] (BP) Definition: The increase in size or mass of the spongiotrophoblast layer of the placenta where the increase in size or mass contributes to the progression of that layer over time from its formation to its mature state. Sources: GOC:dph, GOC:tb Relationships: is_a developmental growth [GO:0048589]; is part of GO:0060712